dCTP deaminase (dUMP-forming) activity [GO:0033973] (MF) Also known as: dCTP aminohydrolase (dUMP-forming) activity Relationships: is a type of hydrolase activity, acting on carbon-nitrogen (but not peptide) bonds, in cyclic amidines [GO:0016814]; is a type of deaminase activity [GO:0019239] Sources: EC:3.5.4.30, RHEA:19205 Definition: Catalysis of the reaction: dCTP + 2 H2O = diphosphate + dUMP + H+ + NH4.